SRP-dependent cotranslational protein targeting to membrane [GO:0006614] (biological process) Relationships: is a type of cotranslational protein targeting to membrane [GO:0006613]; is a type of protein targeting to ER [GO:0045047]; has part translation [GO:0006412] Definition: The targeting of proteins to a membrane that occurs during translation and is dependent upon two key components, the signal-recognition particle (SRP) and the SRP receptor. SRP is a cytosolic particle that transiently binds to the endoplasmic reticulum (ER) signal sequence in a nascent protein, to the large ribosomal unit, and to the SRP receptor in the ER membrane. Sources: ISBN:0716731363 Also known as: ER translocation, SRP-dependent cotranslational membrane targeting, SRP-dependent cotranslational protein-membrane targeting